{
  "term_id": "GO:0043123",
  "gene_symbol": "TRIM13",
  "gene": "UniProtKB:O60858",
  "gene_name": "E3 ubiquitin-protein ligase TRIM13",
  "term_label": "positive regulation of canonical NF-kappaB signal transduction"
}